{
  "gene_name": "Putative annexin A2-like protein",
  "term_id": "GO:0005737",
  "gene_symbol": "ANXA2P2",
  "gene": "UniProtKB:A6NMY6",
  "term_label": "cytoplasm"
}